{
  "gene_symbol": "TRGJ1",
  "gene_name": "T cell receptor gamma joining 1",
  "term_label": "Unknown molecular function",
  "term_id": "UNKNOWN:0001",
  "gene": "UniProtKB:A0A075B6S0"
}